{
  "gene": "UniProtKB:Q5HYJ1",
  "gene_name": "Trans-2,3-enoyl-CoA reductase-like",
  "term_id": "GO:0006665",
  "term_label": "sphingolipid metabolic process",
  "gene_symbol": "TECRL"
}